{
  "term_label": "RNA polymerase II cis-regulatory region sequence-specific DNA binding",
  "gene_symbol": "GLIS2",
  "gene": "UniProtKB:Q9BZE0",
  "gene_name": "Zinc finger protein GLIS2",
  "term_id": "GO:0000978"
}